urea transmembrane transport [GO:0071918] (biological process) Subtypes: urea import across plasma membrane [GO:0140201] Relationships: is a type of GO:0015840; is a type of transmembrane transport [GO:0055085] Also known as: urea membrane transport Note: Note that this term is not intended for use in annotating lateral movement within membranes. Sources: GOC:mah Definition: The process in which urea, the water-soluble compound H2N-CO-NH2, is transported from one side of a membrane to the other by means of some agent such as a transporter or pore.